{
  "term_label": "DNA-binding transcription factor activity, RNA polymerase II-specific",
  "gene": "UniProtKB:Q86TJ5",
  "gene_name": "Zinc finger protein 554",
  "gene_symbol": "ZNF554",
  "term_id": "GO:0000981"
}